prostate field specification [GO:0060515] (biological process) Definition: The process that results in the delineation of a specific region of the urogenital sinus epithelium into the area in which the prostate gland will develop. Relationships: is a type of developmental process involved in reproduction [GO:0003006]; is a type of specification of animal organ identity [GO:0010092]; is part of GO:0060513 Regulation: positively regulated by prostate induction [GO:0060514] References: PMID:18977204 Sources: GOC:dph